{
  "gene": "UniProtKB:Q96J42",
  "term_label": "Unknown molecular function",
  "term_id": "UNKNOWN:0001",
  "gene_name": "Thioredoxin domain-containing protein 15",
  "gene_symbol": "TXNDC15"
}